{
  "term_label": "regulation of gene expression",
  "gene_symbol": "HNRNPD",
  "gene": "UniProtKB:Q14103",
  "gene_name": "Heterogeneous nuclear ribonucleoprotein D0",
  "term_id": "GO:0010468"
}